regulation of spongiotrophoblast cell proliferation [GO:0060721] (biological process) Definition: Any process that modulates the rate, frequency or extent of spongiotrophoblast cell proliferation. Relationships: is a type of GO:0060723; regulates spongiotrophoblast cell proliferation [GO:0060720] Sources: GOC:dph